{
  "gene_name": "Vacuolar protein sorting-associated protein 26B",
  "term_label": "retromer, cargo-selective complex",
  "gene_symbol": "VPS26B",
  "gene": "UniProtKB:Q4G0F5",
  "term_id": "GO:0030906"
}